integrin alpha4-beta1 complex [GO:0034668] (cellular component) Also known as: VLA-4 complex, alpha4-beta1 integrin complex, ITGA4-ITGB1 complex Definition: An integrin complex that comprises one alpha4 subunit and one beta1 subunit. References: PMID:12297042 Relationships: is a type of integrin complex [GO:0008305]